mitotic spindle assembly checkpoint MAD1-MAD2 complex [GO:1990728] (cellular component) Relationships: is a type of GO:0032991; is part of cytoplasm [GO:0005737]; has part GO:1990706 Also known as: MAD1-MAD2 complex Definition: A protein complex involved in the assembly of the mitotic checkpoint complex that in turn inhibits the anaphase promoting complex/cyclosome (APC/C). The MAD1 dimer recruits the open form of MAD2 (O-MAD2) turning it into the closed form (C-MAD2) upon binding. C-MAD2 inhibits CDC20, a member of the APC/C, upon release from the MAD1-MAD2 complex. References: PMID:12006501, PMID:22898774 Sources: GOC:bhm Note: An example of this is MAD1 in human (Q9Y6D9) in PMID:12006501 (inferred from physical interaction).